glycine catabolic process to isobutanol [GO:1902696] (biological process) Definition: The chemical reactions and pathways resulting in the breakdown of glycine to isobutanol. References: PMID:23642236 Sources: GOC:TermGenie, GOC:mengo_curators, GO_REF:0000093 Relationships: is a type of GO:0006546; is a type of GO:0034308 Also known as: glycine breakdown to isobutanol, glycine catabolism to isobutanol, glycine degradation to isobutanol